{
  "gene_name": "Olfactory receptor 4C6",
  "term_label": "olfactory receptor activity",
  "gene": "UniProtKB:Q8NH72",
  "gene_symbol": "OR4C6",
  "term_id": "GO:0004984"
}